{
  "gene_symbol": "CETP",
  "term_label": "phosphatidylcholine binding",
  "gene": "UniProtKB:P11597",
  "term_id": "GO:0031210",
  "gene_name": "Cholesteryl ester transfer protein"
}